{
  "gene_symbol": "ADH1C",
  "gene_name": "Alcohol dehydrogenase 1C",
  "term_label": "all-trans-retinol dehydrogenase (NAD+) activity",
  "gene": "UniProtKB:P00326",
  "term_id": "GO:0004745"
}